{
  "gene": "UniProtKB:P04062",
  "term_id": "GO:0006680",
  "term_label": "glucosylceramide catabolic process",
  "gene_name": "Lysosomal acid glucosylceramidase",
  "gene_symbol": "GBA1"
}